{
  "term_id": "GO:0071333",
  "term_label": "cellular response to glucose stimulus",
  "gene": "UniProtKB:Q16822",
  "gene_name": "Phosphoenolpyruvate carboxykinase [GTP], mitochondrial",
  "gene_symbol": "PCK2"
}